{
  "term_id": "GO:0005634",
  "gene_name": "Oligodendrocyte transcription factor 2",
  "gene": "UniProtKB:Q13516",
  "term_label": "nucleus",
  "gene_symbol": "OLIG2"
}